{
  "gene_symbol": "DPY19L2",
  "gene_name": "Probable C-mannosyltransferase DPY19L2",
  "term_label": "mannosyltransferase activity",
  "gene": "UniProtKB:Q6NUT2",
  "term_id": "GO:0000030"
}